{
  "gene": "UniProtKB:Q5K4L6",
  "gene_symbol": "SLC27A3",
  "gene_name": "Long-chain fatty acid transport protein 3",
  "term_id": "GO:0005886",
  "term_label": "plasma membrane"
}